scaRNA localization to Cajal body [GO:0090666] (biological process) Relationships: is a type of RNA localization to Cajal body [GO:0090670] References: PMID:25467444 Sources: GOC:BHF, GOC:BHF_telomere, GOC:nc Definition: A process in which a small Cajal body-specific RNA is transported to, or maintained in, a Cajal body.